{
  "term_label": "SNAP receptor activity",
  "gene_symbol": "STX3",
  "term_id": "GO:0005484",
  "gene": "UniProtKB:Q13277",
  "gene_name": "Syntaxin-3"
}